{
  "gene": "UniProtKB:Q01518",
  "gene_name": "Adenylyl cyclase-associated protein 1",
  "gene_symbol": "CAP1",
  "term_id": "GO:0008179",
  "term_label": "adenylate cyclase binding"
}